{
  "term_id": "GO:0008013",
  "gene_name": "Cadherin-10",
  "term_label": "beta-catenin binding",
  "gene": "UniProtKB:Q9Y6N8",
  "gene_symbol": "CDH10"
}